{
  "gene": "UniProtKB:Q53EZ4",
  "gene_symbol": "CEP55",
  "term_id": "UNKNOWN:0001",
  "term_label": "Unknown molecular function",
  "gene_name": "Centrosomal protein of 55 kDa"
}